GUU codon-amino acid adaptor activity [GO:0033449] (molecular function) Definition: A triplet codon-amino acid adaptor activity that recognizes a GUU codon. Relationships: is a type of triplet codon-amino acid adaptor activity [GO:0030533] Note: Note that in the standard genetic code, GTT codes for valine. Sources: GOC:mah Also known as: GTT codon-amino acid adaptor activity, valine tRNA